{
  "term_label": "Unknown cellular component",
  "gene_symbol": "PRR23D1",
  "gene": "UniProtKB:E9PI22",
  "term_id": "UNKNOWN:0003",
  "gene_name": "Proline-rich protein 23D1"
}